{
  "gene_symbol": "TUBA3E",
  "term_id": "GO:0000226",
  "gene": "UniProtKB:Q6PEY2",
  "term_label": "microtubule cytoskeleton organization",
  "gene_name": "Tubulin alpha-3E chain"
}